DNA replication [GO:0006260] (biological process) Regulation: regulated by regulation of DNA replication [GO:0006275]; negatively regulated by negative regulation of DNA replication [GO:0008156]; positively regulated by GO:0045740 Subtypes: DNA-templated DNA replication [GO:0006261] Definition: The cellular metabolic process in which a cell duplicates one or more molecules of DNA. DNA replication begins when specific sequences, known as origins of replication, are recognized and bound by the origin recognition complex, and ends when the original DNA molecule has been completely duplicated and the copies topologically separated. The unit of replication usually corresponds to the genome of the cell, an organelle, or a virus. The template for replication can either be an existing DNA molecule or RNA. Relationships: is a type of DNA metabolic process [GO:0006259]; has part DNA biosynthetic process [GO:0071897] Note: DNA biosynthesis is only part of this process. See also the biological process terms 'DNA-dependent DNA replication ; GO:0006261' and 'RNA-dependent DNA replication ; GO:0006278'. Sources: GOC:mah